vitamin K catabolic process [GO:0042377] (biological process) Also known as: naphthoquinone catabolic process, naphthoquinone catabolism, vitamin K breakdown, vitamin K catabolism, vitamin K degradation Relationships: is a type of ketone catabolic process [GO:0042182]; is a type of fat-soluble vitamin catabolic process [GO:0042363]; is a type of vitamin K metabolic process [GO:0042373] References: PMID:24489112 Sources: GOC:jl, https://en.wikipedia.org/wiki/Vitamin_K Subtypes: phylloquinone catabolic process [GO:0042376] Definition: The chemical reactions and pathways resulting in the breakdown of any of the forms of vitamin K, quinone-derived vitamins which are involved in the synthesis of blood-clotting factors in mammals.